{
  "gene_name": "Small regulatory polypeptide of amino acid response",
  "term_label": "Unknown molecular function",
  "gene": "UniProtKB:A0A1B0GVQ0",
  "term_id": "UNKNOWN:0001",
  "gene_symbol": "SPAAR"
}